basidium development [GO:0075313] (biological process) Regulation: regulated by regulation of basidium development [GO:0075314]; positively regulated by GO:0075315; negatively regulated by negative regulation of basidium development [GO:0075316] Definition: The process that leads to the development of basidium, a small, specialized club-shaped structure typically bearing four basidiospores at the tips of minute projections. The basidium is unique to Basidiomycetes and distinguishes them from other kinds of fungi. Relationships: is a type of spore-bearing structure development [GO:0075259] Sources: GOC:di, GOC:mah, GOC:mcc, GOC:pamgo_curators Note: Note that basidiospores and basidia are separate biological structures. The basidium is the structure that bear the basidiospores, but the development of the basidium is a different process than the formation of the basidiospores themselves. For this reason, GO:0034295 basidiospore formation and GO:0075313 basidium development are different terms and are not linked.